{
  "term_id": "GO:0005615",
  "gene": "UniProtKB:Q9UKR3",
  "term_label": "extracellular space",
  "gene_symbol": "KLK13",
  "gene_name": "Kallikrein-13"
}